raps-insc complex [GO:1990499] (cellular component) Definition: Protein complex required for the asymmetric division of neuroblasts in Drosophila. Coordinates asymmetric localization of cell fate determinants with orientation of the mitotic spindle resulting in different daughter cells upon division. Localizes at the apical cortex of the neuroblast: Raps maintains, but does not initiate, Insc apically, while Insc segregates Raps asymmetrically. Complex appears to be conserved in mammals (composed of INSC and GPSM1 or GPSM2). References: PMID:22171003 Sources: GOC:bhm Also known as: Rapsynoid-Inscuteable complex, partner of inscuteable-inscuteable complex Note: An example of this is Insc in drome (Q9W2R4) in PMID:22171003 (inferred from physical interaction). Relationships: is a type of protein-containing complex [GO:0032991]; is part of apical cortex [GO:0045179]